protein transport along microtubule to kinetochore [GO:0140210] (biological process) Definition: Any process in which a protein is transported to the kinetochore along a microtubule. References: PMID:25472718 Relationships: is a type of protein localization to kinetochore [GO:0034501]; is a type of establishment of protein localization to chromosome [GO:0070199]; is a type of protein transport along microtubule [GO:0098840]